{
  "gene_symbol": "SPATA16",
  "gene": "UniProtKB:Q9BXB7",
  "term_label": "Golgi apparatus",
  "gene_name": "Spermatogenesis-associated protein 16",
  "term_id": "GO:0005794"
}